{
  "gene_symbol": "ITGA9",
  "term_label": "integrin alpha9-beta1 complex",
  "gene": "UniProtKB:Q13797",
  "term_id": "GO:0034679",
  "gene_name": "Integrin alpha-9"
}